{
  "term_label": "nucleus",
  "gene_name": "NMDA receptor synaptonuclear signaling and neuronal migration factor",
  "gene": "UniProtKB:Q6X4W1",
  "gene_symbol": "NSMF",
  "term_id": "GO:0005634"
}